{
  "gene_symbol": "METTL21C",
  "gene_name": "Protein-lysine methyltransferase METTL21C",
  "gene": "UniProtKB:Q5VZV1",
  "term_id": "GO:0008276",
  "term_label": "protein methyltransferase activity"
}